{
  "term_id": "GO:0006955",
  "gene_name": "Asialoglycoprotein receptor 1",
  "term_label": "immune response",
  "gene_symbol": "ASGR1",
  "gene": "UniProtKB:P07306"
}